{
  "gene_name": "DNA (cytosine-5)-methyltransferase 3A",
  "term_id": "GO:0005634",
  "gene": "UniProtKB:Q9Y6K1",
  "gene_symbol": "DNMT3A",
  "term_label": "nucleus"
}